{
  "gene_name": "Contactin-associated protein-like 2",
  "term_label": "signal transduction",
  "term_id": "GO:0007165",
  "gene": "UniProtKB:Q9UHC6",
  "gene_symbol": "CNTNAP2"
}